positive regulation of detection of glucose [GO:2000972] (biological process) Relationships: is a type of GO:0048584; is a type of regulation of detection of glucose [GO:2000970]; positively regulates detection of glucose [GO:0051594] Definition: Any process that activates or increases the frequency, rate or extent of detection of glucose. Also known as: positive regulation of glucose detection, positive regulation of glucose perception, positive regulation of glucose sensing Sources: GOC:BHF